{
  "term_id": "GO:0031640",
  "gene_symbol": "GNLY",
  "gene_name": "Granulysin",
  "term_label": "killing of cells of another organism",
  "gene": "UniProtKB:P22749"
}